laminin-2 complex [GO:0005607] (cellular component) Definition: A laminin complex composed of alpha2, beta1 and gamma1 polypeptide chains. References: PMID:10842354 Sources: GOC:jl Also known as: laminin-211 complex Relationships: is a type of GO:0043256